{
  "gene_name": "Zinc finger and BTB domain-containing protein 11",
  "term_label": "RNA polymerase II cis-regulatory region sequence-specific DNA binding",
  "term_id": "GO:0000978",
  "gene_symbol": "ZBTB11",
  "gene": "UniProtKB:O95625"
}